{
  "term_label": "Unknown molecular function",
  "gene_symbol": "MRPL9",
  "gene": "UniProtKB:Q9BYD2",
  "term_id": "UNKNOWN:0001",
  "gene_name": "Large ribosomal subunit protein bL9m"
}